{
  "term_label": "Unknown cellular component",
  "gene_name": "Beta-1,3-galactosyl-O-glycosyl-glycoprotein beta-1,6-N-acetylglucosaminyltransferase 7",
  "term_id": "UNKNOWN:0003",
  "gene_symbol": "GCNT7",
  "gene": "UniProtKB:Q6ZNI0"
}